{
  "gene": "UniProtKB:O95711",
  "term_label": "positive regulation of lipopolysaccharide-mediated signaling pathway",
  "gene_name": "Lymphocyte antigen 86",
  "term_id": "GO:0031666",
  "gene_symbol": "LY86"
}